{
  "term_id": "UNKNOWN:0001",
  "gene": "UniProtKB:Q96LS8",
  "term_label": "Unknown molecular function",
  "gene_name": "Putative uncharacterized protein C2orf48",
  "gene_symbol": "C2orf48"
}